neck portion of tanycyte [GO:1990016] (CC) Sources: ISBN:0195065719, NIF_Subcellular:sao901230115 Also known as: neck portion Definition: Elongated portion of a tanycyte that sticks into the periventricular layer of neuropil where it appears to contact a blood vessel; characterized by numerous cytoplasmic extensions. A tanycyte is a specialized elongated ventricular ependymal cell that has processes that extend to the outer, or pial, surface of the CNS. Relationships: is a type of cellular anatomical structure [GO:0110165]